PSII associated light-harvesting complex II, core complex [GO:0009655] (CC) Sources: GOC:lr Relationships: is a type of chloroplast thylakoid membrane protein complex [GO:0098807]; is part of PSII associated light-harvesting complex II [GO:0009517] Also known as: PSII associated light-harvesting complex II, core complex, LHCIIa subcomplex, PSII associated light-harvesting complex II, core complex, LHCIIc subcomplex, PSII associated light-harvesting complex II, core complex, LHCIId subcomplex Definition: The pigment-protein complex primarily associated to PSII in higher plants, green algae and cyanobacteria that directly transfers electrons to the reaction center.